latrotoxin receptor activity [GO:0016524] (molecular function) Relationships: is a type of transmembrane signaling receptor activity [GO:0004888] Definition: Combining with alpha-latrotoxin, a potent presynaptic neurotoxin, and transmitting the signal from one side of the membrane to the other to initiate a change in cell activity. Also known as: latrophilin References: PMID:10025961 Sources: GOC:jl, GOC:signaling